{
  "term_id": "GO:0035402",
  "gene_symbol": "CHEK1",
  "gene": "UniProtKB:O14757",
  "gene_name": "Serine_threonine-protein kinase Chk1",
  "term_label": "histone H3T11 kinase activity"
}